{
  "gene": "UniProtKB:Q9UL17",
  "term_label": "regulation of transcription by RNA polymerase II",
  "gene_name": "T-box transcription factor TBX21",
  "gene_symbol": "TBX21",
  "term_id": "GO:0006357"
}